{
  "term_id": "GO:0006357",
  "gene": "UniProtKB:Q7Z5L9",
  "term_label": "regulation of transcription by RNA polymerase II",
  "gene_symbol": "IRF2BP2",
  "gene_name": "Interferon regulatory factor 2-binding protein 2"
}